{
  "gene": "UniProtKB:Q9NQY0",
  "gene_symbol": "BIN3",
  "term_label": "actin cortical patch localization",
  "term_id": "GO:0051666",
  "gene_name": "Bridging integrator 3"
}